{
  "term_label": "Unknown molecular function",
  "term_id": "UNKNOWN:0001",
  "gene": "UniProtKB:Q8N910",
  "gene_name": "Putative uncharacterized protein PAK6-AS1",
  "gene_symbol": "PAK6-AS1"
}